{
  "gene": "UniProtKB:Q5T8D3",
  "term_label": "cytoplasm",
  "gene_name": "Acyl-CoA-binding domain-containing protein 5",
  "term_id": "GO:0005737",
  "gene_symbol": "ACBD5"
}